oligo-1,6-glucosidase activity [GO:0004574] (molecular function) Definition: Catalysis of the hydrolysis of (1->6)-alpha-D-glucosidic linkages in some oligosaccharides produced from starch and glycogen by alpha-amylase, and in isomaltose. Releases a free alpha-D-glucose. Sources: EC:3.2.1.10 Relationships: is_a alpha-glucosidase activity [GO:0090599] Also known as: alpha-limit dextrinase activity, alpha-methylglucosidase activity, dextrin 6-glucanohydrolase activity, dextrin 6alpha-glucanohydrolase activity, exo-oligo-1,6-glucosidase activity, isomaltase activity, limit dextrinase, oligosaccharide alpha-1,6-glucohydrolase activity, oligosaccharide alpha-1,6-glucosidase activity, sucrase-isomaltase activity